{
  "term_label": "Unknown molecular function",
  "term_id": "UNKNOWN:0001",
  "gene_name": "Sperm axonemal maintenance protein CFAP97D1",
  "gene_symbol": "CFAP97D1",
  "gene": "UniProtKB:B2RV13"
}